{
  "term_id": "GO:0005737",
  "gene_name": "Probable E3 ubiquitin-protein ligase TRIML1",
  "gene": "UniProtKB:Q8N9V2",
  "gene_symbol": "TRIML1",
  "term_label": "cytoplasm"
}